{
  "term_id": "GO:0050808",
  "gene_name": "Contactin-4",
  "gene_symbol": "CNTN4",
  "gene": "UniProtKB:Q8IWV2",
  "term_label": "synapse organization"
}